{
  "gene_symbol": "NLGN3",
  "gene_name": "Neuroligin-3",
  "term_id": "GO:0050804",
  "term_label": "modulation of chemical synaptic transmission",
  "gene": "UniProtKB:Q9NZ94"
}